{
  "term_label": "centrosome",
  "gene_symbol": "TUBG1",
  "gene": "UniProtKB:P23258",
  "gene_name": "Tubulin gamma-1 chain",
  "term_id": "GO:0005813"
}